{
  "gene_symbol": "NCAN",
  "gene_name": "Neurocan core protein",
  "term_label": "Unknown molecular function",
  "term_id": "UNKNOWN:0001",
  "gene": "UniProtKB:O14594"
}